{
  "term_label": "lipid homeostasis",
  "gene": "UniProtKB:Q8N8W4",
  "term_id": "GO:0055088",
  "gene_symbol": "PNPLA1",
  "gene_name": "Omega-hydroxyceramide transacylase"
}